clathrin-dependent synaptic vesicle endocytosis [GO:0150007] (biological process) Definition: Clathrin-dependent endocytosis of presynaptic membrane regions comprising synaptic vesicles' membrane constituents. This is a relatively slow process occurring in the range of tens of seconds. References: PMID:16982422, PMID:18579735, PMID:18579748, PMID:26430111, PMID:27252645, PMID:28391090, PMID:4348786 Sources: GOC:aruk, GOC:bc, GOC:ha Relationships: is a type of intracellular transport [GO:0046907]; is a type of synaptic vesicle endocytosis [GO:0048488]; is a type of clathrin-dependent endocytosis [GO:0072583]; is part of GO:0036466